{
  "gene": "UniProtKB:P25391",
  "term_label": "basement membrane",
  "gene_name": "Laminin subunit alpha-1",
  "term_id": "GO:0005604",
  "gene_symbol": "LAMA1"
}